{
  "gene": "UniProtKB:Q8IV36",
  "gene_symbol": "HID1",
  "gene_name": "Protein HID1",
  "term_id": "GO:0016020",
  "term_label": "membrane"
}